{
  "term_label": "cell differentiation",
  "term_id": "GO:0030154",
  "gene_name": "Forkhead box protein B2",
  "gene": "UniProtKB:Q5VYV0",
  "gene_symbol": "FOXB2"
}